symbiont-mediated perturbation of host vacuole organization [GO:0044075] (biological process) Definition: A process in which a symbiont alters or subverts vacuole organization in its host organism. The host is defined as the larger of the organisms involved in a symbiotic interaction. Also known as: modulation by symbiont of host vacuole organisation, modulation by symbiont of host vacuole organization, modulation of host vacuole organization by symbiont, regulation by symbiont of host vacuole organization, modulation by symbiont of host vacuole biogenesis Subtypes: symbiont-mediated generation of symbiont replication vacuole [GO:0141213] References: PMID:25139904 Relationships: is a type of symbiont-mediated perturbation of host cellular process [GO:0044068]